double-stranded RNA adenosine deaminase activity [GO:0003726] (molecular function) Definition: Catalysis of the reaction: adenosine + H2O = inosine + NH3, in a double-stranded RNA molecule. Sources: GOC:mah, RHEA:10120 Also known as: double-stranded RNA specific editase activity Relationships: is_a GO:0019239